{
  "gene": "UniProtKB:Q96EE4",
  "gene_symbol": "CCDC126",
  "gene_name": "Coiled-coil domain-containing protein 126",
  "term_label": "Unknown cellular component",
  "term_id": "UNKNOWN:0003"
}